aspartate binding [GO:0070335] (molecular function) Also known as: aspartic acid binding Sources: CHEBI:29995, GOC:mah Definition: Binding to aspartate, the alpha-amino-acid anion of 2-aminobutanedioic acid that has formula C4H5NO4. Relationships: is a type of amino acid binding [GO:0016597]; is a type of GO:0031406